{
  "term_id": "GO:0005886",
  "term_label": "plasma membrane",
  "gene": "UniProtKB:P21926",
  "gene_symbol": "CD9",
  "gene_name": "CD9 antigen"
}